cone photoreceptor outer segment [GO:0120199] (CC) Definition: The outer segment of a vertebrate cone photoreceptor that contains membrane discs that are contiguous with the ciliary membrane and containing opsin photoreceptor proteins. Relationships: is a type of photoreceptor outer segment [GO:0001750] References: PMID:19501669, PMID:26574505, PMID:6771304 Sources: GOC:krc, GOC:pde